{
  "gene": "UniProtKB:Q8IVH8",
  "term_id": "GO:0008349",
  "term_label": "MAP kinase kinase kinase kinase activity",
  "gene_name": "Mitogen-activated protein kinase kinase kinase kinase 3",
  "gene_symbol": "MAP4K3"
}